cyanelle intermembrane space [GO:0036014] (cellular component) Sources: GOC:aa Definition: The region between the inner and outer lipid bilayers of the cyanelle envelope; includes the peptidoglycan layer. Also known as: cyanelle envelope lumen, cyanelle periplasm Relationships: is a type of GO:0009529; is part of cyanelle envelope [GO:0033112]